vinculin binding [GO:0017166] (molecular function) Sources: ISBN:0721662544 Relationships: is_a GO:0008092 Definition: Binding to vinculin, a protein found in muscle, fibroblasts, and epithelial cells that binds actin and appears to mediate attachment of actin filaments to integral proteins of the plasma membrane.